spermine synthase activity [GO:0016768] (molecular function) Also known as: S-adenosylmethioninamine:spermidine 3-aminopropyltransferase activity, spermidine aminopropyltransferase activity, spermine synthetase activity Sources: EC:2.5.1.22 Relationships: is a type of GO:0016765 Definition: Catalysis of the reaction: S-adenosylmethioninamine + spermidine = 5'-methylthioadenosine + spermine.